regulation of post-lysosomal vacuole size [GO:0044656] (biological process) Relationships: is a type of regulation of vesicle size [GO:0097494] References: PMID:22008230 Sources: GOC:rjd Definition: Any process that modulates the volume of a post-lysosomal vacuole, a membrane-bounded intracellular vesicle formed late in the endocytic pathway when the pH in the vacuole becomes neutral prior to exocytosis. Also known as: regulation of post-lysosome size, regulation of postlysosomal vacuole size, regulation of postlysosome vacuole size